{
  "gene_name": "Dual specificity protein phosphatase 10",
  "term_label": "MAP kinase tyrosine phosphatase activity",
  "gene": "UniProtKB:Q9Y6W6",
  "gene_symbol": "DUSP10",
  "term_id": "GO:0033550"
}